{
  "term_label": "elongator holoenzyme complex",
  "gene_name": "Elongator complex protein 3",
  "term_id": "GO:0033588",
  "gene": "UniProtKB:Q9H9T3",
  "gene_symbol": "ELP3"
}